{
  "term_label": "unfolded protein binding",
  "gene_name": "DnaJ homolog subfamily B member 11",
  "gene_symbol": "DNAJB11",
  "gene": "UniProtKB:Q9UBS4",
  "term_id": "GO:0051082"
}